{
  "term_id": "UNKNOWN:0003",
  "gene_symbol": "DOHH",
  "gene": "UniProtKB:Q9BU89",
  "term_label": "Unknown cellular component",
  "gene_name": "Deoxyhypusine hydroxylase"
}